{
  "gene_symbol": "DUSP13B",
  "gene": "UniProtKB:Q9UII6",
  "term_label": "MAP kinase phosphatase activity",
  "term_id": "GO:0033549",
  "gene_name": "Dual specificity protein phosphatase 13 isoform B"
}